{
  "term_id": "UNKNOWN:0003",
  "term_label": "Unknown cellular component",
  "gene_symbol": "CHIC1",
  "gene_name": "Cysteine-rich hydrophobic domain-containing protein 1",
  "gene": "UniProtKB:Q5VXU3"
}